{
  "term_label": "hepoxilin biosynthetic process",
  "gene_symbol": "ALOX12B",
  "gene_name": "Arachidonate 12-lipoxygenase, 12R-type",
  "gene": "UniProtKB:O75342",
  "term_id": "GO:0051122"
}